regulation of establishment of RNA localization to telomere [GO:1904910] (biological process) References: PMID:26586433 Sources: GOC:BHF, GOC:BHF_telomere, GOC:TermGenie, GOC:rph, GO_REF:0000058 Subtypes: GO:1904911, GO:1904912 Also known as: regulation of establishment of RNA localisation to telomere Relationships: is a type of regulation of localization [GO:0032879]; RO_0002211 establishment of RNA localization to telomere [GO:0097694] Definition: Any process that modulates the frequency, rate or extent of establishment of RNA localization to telomere.